{
  "gene_name": "Uncharacterized protein FLJ37310",
  "gene": "UniProtKB:Q8N1X5",
  "term_label": "Unknown cellular component",
  "gene_symbol": "Q8N1X5",
  "term_id": "UNKNOWN:0003"
}